{
  "term_id": "GO:0003713",
  "term_label": "transcription coactivator activity",
  "gene_name": "Transcription initiation factor TFIID subunit 6",
  "gene": "UniProtKB:P49848",
  "gene_symbol": "TAF6"
}